{
  "gene_name": "Protein argonaute-1",
  "gene": "UniProtKB:Q9UL18",
  "term_label": "pre-miRNA processing",
  "term_id": "GO:0031054",
  "gene_symbol": "AGO1"
}